{
  "term_label": "6-phosphofructo-2-kinase/fructose-2,6-biphosphatase complex",
  "gene_name": "6-phosphofructo-2-kinase_fructose-2,6-bisphosphatase 1",
  "gene": "UniProtKB:P16118",
  "term_id": "GO:0043540",
  "gene_symbol": "PFKFB1"
}